{
  "term_label": "cell-cell junction",
  "gene": "UniProtKB:Q8IZU9",
  "term_id": "GO:0005911",
  "gene_name": "Kin of IRRE-like protein 3",
  "gene_symbol": "KIRREL3"
}